{
  "term_label": "plasma membrane",
  "gene": "UniProtKB:Q8NC01",
  "term_id": "GO:0005886",
  "gene_symbol": "CLEC1A",
  "gene_name": "C-type lectin domain family 1 member A"
}